positive regulation of T cell differentiation in thymus [GO:0033089] (biological process) Also known as: positive regulation of thymic T cell differentiation, positive regulation of thymocyte cell differentiation, positive regulation of thymocyte differentiation, positive regulation of T cell development in thymus Subtypes: positive regulation of positive thymic T cell selection [GO:1902234] Relationships: is a type of GO:0033081; is a type of positive regulation of T cell differentiation [GO:0045582]; positively regulates T cell differentiation in thymus [GO:0033077] Sources: GOC:add, GOC:mah Definition: Any process that activates or increases the frequency, rate or extent of T cell differentiation in the thymus. Note: Note that immunologists typically use the word 'development' to refer to cells of B or T cell lineages undergoing the process that GO describes as 'cell differentiation'.